{
  "gene_name": "Fibrous sheath-interacting protein 2",
  "gene_symbol": "FSIP2",
  "term_label": "Unknown molecular function",
  "gene": "UniProtKB:Q5CZC0",
  "term_id": "UNKNOWN:0001"
}